{
  "term_id": "GO:0015204",
  "term_label": "urea transmembrane transporter activity",
  "gene_name": "Aquaporin-3",
  "gene": "UniProtKB:Q92482",
  "gene_symbol": "AQP3"
}